positive regulation of respiratory burst [GO:0060267] (biological process) Subtypes: positive regulation of respiratory burst involved in inflammatory response [GO:0060265] Relationships: is a type of positive regulation of metabolic process [GO:0009893]; is a type of regulation of respiratory burst [GO:0060263]; positively regulates respiratory burst [GO:0045730] Definition: Any process that increases the rate frequency or extent of a phase of elevated metabolic activity, during which oxygen consumption increases; this leads to the production, by an NADH dependent system, of hydrogen peroxide (H2O2), superoxide anions and hydroxyl radicals. Sources: GOC:dph, GOC:tb